{
  "term_id": "GO:0005886",
  "gene_name": "Potassium channel subfamily K member 9",
  "gene_symbol": "KCNK9",
  "term_label": "plasma membrane",
  "gene": "UniProtKB:Q9NPC2"
}